{
  "term_label": "dendritic cell differentiation",
  "gene_symbol": "LYN",
  "gene": "UniProtKB:P07948",
  "term_id": "GO:0097028",
  "gene_name": "Tyrosine-protein kinase Lyn"
}